cellular response to mercaptoethanol [GO:0072705] (biological process) Definition: Any process that results in a change in state or activity of a cell (in terms of movement, secretion, enzyme production, gene expression, etc.) as a result of a mercaptoethanol stimulus. Also known as: cellular response to 2-sulfanylethanol Sources: GOC:mah Relationships: is a type of response to mercaptoethanol [GO:0072704]; is a type of cellular response to alcohol [GO:0097306]